{
  "gene_symbol": "CHMP4B",
  "gene": "UniProtKB:Q9H444",
  "term_id": "GO:0009898",
  "gene_name": "Charged multivesicular body protein 4b",
  "term_label": "cytoplasmic side of plasma membrane"
}